phosphoserine:homoserine phosphotransferase activity [GO:0043899] (molecular function) Relationships: is_a phosphotransferase activity, alcohol group as acceptor [GO:0016773] Definition: Catalysis of the transfer of a phosphoryl group from phosphoserine to homoserine to form phosphohomoserine. Also known as: thrH References: PMID:14699121 Sources: GOC:jl